{
  "gene_symbol": "MAD1L1",
  "gene_name": "Mitotic spindle assembly checkpoint protein MAD1",
  "term_label": "attachment of mitotic spindle microtubules to kinetochore",
  "term_id": "GO:0051315",
  "gene": "UniProtKB:Q9Y6D9"
}